{
  "term_id": "UNKNOWN:0001",
  "gene": "UniProtKB:Q6UWK7",
  "gene_symbol": "GPR15L",
  "gene_name": "Protein GPR15LG",
  "term_label": "Unknown molecular function"
}